{
  "gene": "UniProtKB:Q86UY6",
  "gene_name": "N-alpha-acetyltransferase 40",
  "gene_symbol": "NAA40",
  "term_id": "GO:1990189",
  "term_label": "protein N-terminal-serine acetyltransferase activity"
}